bicyclogermacrene catabolic process [GO:1901933] (biological process) Also known as: bicyclogermacrene breakdown, bicyclogermacrene catabolism, bicyclogermacrene degradation References: PMID:22867794 Sources: GOC:TermGenie Relationships: is_a sesquiterpene catabolic process [GO:0051763] Definition: The chemical reactions and pathways resulting in the breakdown of bicyclogermacrene.